{
  "term_label": "proteolysis",
  "gene": "UniProtKB:Q14520",
  "gene_symbol": "HABP2",
  "gene_name": "Hyaluronan-binding protein 2",
  "term_id": "GO:0006508"
}